{
  "term_id": "UNKNOWN:0003",
  "gene_symbol": "TEX53",
  "gene_name": "Testis-expressed protein 53",
  "term_label": "Unknown cellular component",
  "gene": "UniProtKB:A0A1B0GU33"
}